{
  "term_label": "cytosol",
  "term_id": "GO:0005829",
  "gene_name": "Ubiquitin carboxyl-terminal hydrolase 17-like protein 21",
  "gene": "UniProtKB:D6R901",
  "gene_symbol": "USP17L21"
}